{
  "term_id": "GO:0032979",
  "gene_symbol": "OXA1L",
  "gene": "UniProtKB:Q15070",
  "gene_name": "Mitochondrial inner membrane protein OXA1L",
  "term_label": "protein insertion into mitochondrial inner membrane from matrix"
}